{
  "gene_symbol": "TRGC2",
  "term_id": "UNKNOWN:0002",
  "term_label": "Unknown biological process",
  "gene": "UniProtKB:P03986",
  "gene_name": "T cell receptor gamma constant 2"
}